{
  "gene": "UniProtKB:P31040",
  "gene_name": "Succinate dehydrogenase [ubiquinone] flavoprotein subunit, mitochondrial",
  "term_label": "succinate dehydrogenase (quinone) activity",
  "term_id": "GO:0008177",
  "gene_symbol": "SDHA"
}